{
  "gene_symbol": "PRO0255",
  "gene_name": "Putative uncharacterized protein PRO0255",
  "term_id": "UNKNOWN:0002",
  "gene": "UniProtKB:Q9UI72",
  "term_label": "Unknown biological process"
}